{
  "term_id": "GO:0042393",
  "gene_symbol": "ATAD2B",
  "gene": "UniProtKB:Q9ULI0",
  "term_label": "histone binding",
  "gene_name": "ATPase family AAA domain-containing protein 2B"
}